positive regulation of lipoprotein particle clearance [GO:0010986] (biological process) Relationships: is a type of regulation of lipoprotein particle clearance [GO:0010984]; is a type of GO:0051240; positively regulates plasma lipoprotein particle clearance [GO:0034381] Definition: Any process that increases the rate, frequency, or extent of lipoprotein particle clearance. Lipoprotein particle clearance is the process in which a lipoprotein particle is removed from the blood via receptor-mediated endocytosis and its constituent parts degraded. Sources: GOC:BHF, GOC:dph, GOC:tb Subtypes: positive regulation of high-density lipoprotein particle clearance [GO:0010983], positive regulation of chylomicron remnant clearance [GO:0090321], positive regulation of very-low-density lipoprotein particle clearance [GO:0110119], GO:1905581